{
  "gene": "UniProtKB:P0C7P3",
  "gene_name": "Protein SLFN14",
  "gene_symbol": "SLFN14",
  "term_id": "GO:0043022",
  "term_label": "ribosome binding"
}